{
  "term_label": "Unknown cellular component",
  "gene_name": "Sperm protein associated with the nucleus on the X chromosome N1",
  "term_id": "UNKNOWN:0003",
  "gene_symbol": "SPANXN1",
  "gene": "UniProtKB:Q5VSR9"
}